{
  "term_label": "tRNA guanylyltransferase activity",
  "gene_symbol": "THG1L",
  "gene_name": "Probable tRNA(His) guanylyltransferase",
  "term_id": "GO:0008193",
  "gene": "UniProtKB:Q9NWX6"
}